acetylgalactosaminyltransferase activity [GO:0008376] (MF) Relationships: is a type of UDP-glycosyltransferase activity [GO:0008194]; is a type of GO:0016758 Also known as: GalNAc transferase activity Sources: ISBN:0198506732 Subtypes: GO:0003947, GO:0004380, polypeptide N-acetylgalactosaminyltransferase activity [GO:0004653], N-acetyl-beta-glucosaminyl-derivative 4-beta-N-acetylgalactosaminyltransferase activity [GO:0033842], alpha-1,4-N-acetylgalactosaminyltransferase activity [GO:0035248], N-acetylneuraminylgalactosylglucosylceramide beta-1,4-N-acetylgalactosaminyltransferase activity [GO:0047233], glucuronylgalactosylproteoglycan 4-beta-N-acetylgalactosaminyltransferase activity [GO:0047237], glucuronosyl-N-acetylgalactosaminyl-proteoglycan 4-beta-N-acetylgalactosaminyltransferase activity [GO:0047238], galactosylgalactosylglucosylceramide beta-D-acetylgalactosaminyltransferase activity [GO:0047273], GO:0047277 Definition: Catalysis of the transfer of an N-acetylgalactosaminyl residue from UDP-N-acetyl-galactosamine to an oligosaccharide.